{
  "gene_symbol": "MRAP",
  "gene": "UniProtKB:Q8TCY5",
  "term_id": "GO:0031782",
  "gene_name": "Melanocortin-2 receptor accessory protein",
  "term_label": "type 4 melanocortin receptor binding"
}